{
  "term_label": "voltage-gated sodium channel complex",
  "gene": "UniProtKB:Q9UQD0",
  "gene_name": "Sodium channel protein type 8 subunit alpha",
  "gene_symbol": "SCN8A",
  "term_id": "GO:0001518"
}